intercellular canaliculus [GO:0046581] (cellular component) Definition: An extremely narrow tubular channel located between adjacent cells. An instance of this is the secretory canaliculi occurring between adjacent parietal cells in the gastric mucosa of vertebrates. Relationships: is a type of cell-cell junction [GO:0005911] Sources: ISBN:0721662544